{
  "gene_name": "Transcription factor 7-like 1",
  "term_id": "GO:0060070",
  "gene": "UniProtKB:Q9HCS4",
  "term_label": "canonical Wnt signaling pathway",
  "gene_symbol": "TCF7L1"
}